B cell adhesion [GO:0097323] (biological process) Definition: The attachment of a B cell to another cell via adhesion molecules. Sources: GOC:jc Relationships: is a type of GO:0007159